{
  "gene_symbol": "SLU7",
  "term_id": "GO:0005681",
  "gene_name": "Pre-mRNA-splicing factor SLU7",
  "term_label": "spliceosomal complex",
  "gene": "UniProtKB:O95391"
}